{
  "term_label": "cell adhesion molecule binding",
  "gene_symbol": "PCDHGA9",
  "gene": "UniProtKB:Q9Y5G4",
  "gene_name": "Protocadherin gamma-A9",
  "term_id": "GO:0050839"
}